{
  "gene_name": "GRB2-associated-binding protein 3",
  "term_id": "GO:0005737",
  "gene_symbol": "GAB3",
  "gene": "UniProtKB:Q8WWW8",
  "term_label": "cytoplasm"
}